{
  "gene_symbol": "SPDYE14",
  "term_id": "UNKNOWN:0002",
  "term_label": "Unknown biological process",
  "gene_name": "Putative speedy protein E14",
  "gene": "UniProtKB:P0DUD3"
}